{
  "term_label": "DNA-binding transcription repressor activity, RNA polymerase II-specific",
  "term_id": "GO:0001227",
  "gene_name": "Adipocyte enhancer-binding protein 1",
  "gene_symbol": "AEBP1",
  "gene": "UniProtKB:Q8IUX7"
}